{
  "term_id": "GO:0008528",
  "gene_symbol": "VIPR1",
  "gene": "UniProtKB:P32241",
  "term_label": "G protein-coupled peptide receptor activity",
  "gene_name": "Vasoactive intestinal polypeptide receptor 1"
}